pheophorbidase activity [GO:0035560] (molecular function) Also known as: PPD activity, phedase activity, pheophoridase activity References: PMID:16228561 Sources: RHEA:32483 Relationships: is a type of carboxylic ester hydrolase activity [GO:0052689] Definition: Catalysis of the reaction: pheophorbide a + H2O = pyropheophorbide a + methanol + CO2. The reaction occurs in two steps; pheophoridase catalyzes the conversion of pheophorbide a to a precursor of pyropheophorbide a, C-13(2)-carboxylpyropheophorbide a, by demethylation, and then the precursor is decarboxylated non-enzymatically to yield pyropheophorbide a.